{
  "term_label": "positive regulation of skeletal muscle fiber development",
  "gene": "UniProtKB:P15172",
  "term_id": "GO:0048743",
  "gene_symbol": "MYOD1",
  "gene_name": "Myoblast determination protein 1"
}